{
  "term_label": "Unknown molecular function",
  "term_id": "UNKNOWN:0001",
  "gene_name": "DEP domain-containing protein 7",
  "gene": "UniProtKB:Q96QD5",
  "gene_symbol": "DEPDC7"
}